{
  "term_id": "GO:1990825",
  "gene_name": "Shiftless antiviral inhibitor of ribosomal frameshifting protein",
  "term_label": "sequence-specific mRNA binding",
  "gene_symbol": "SHFL",
  "gene": "UniProtKB:Q9NUL5"
}